intracellular arginine homeostasis [GO:0090465] (BP) Also known as: arginine homeostasis, cellular arginine homeostasis Sources: GOC:tb Definition: A homeostatic process involved in the maintenance of a steady state level of arginine within a cell. Relationships: is a type of GO:0080144